{
  "term_label": "calcium ion sensor activity",
  "gene_name": "Synaptotagmin-17",
  "gene": "UniProtKB:Q9BSW7",
  "term_id": "GO:0061891",
  "gene_symbol": "SYT17"
}